transcription coactivator activity [GO:0003713] (molecular function) Note: For usage guidance, see comment in GO:0003712 ; transcription coregulator activity. Relationships: is_a transcription coregulator activity [GO:0003712]; is part of positive regulation of DNA-templated transcription [GO:0045893] Definition: A transcription coregulator activity that activates or increases the transcription of specific gene sets via binding to a DNA-binding transcription factor at a specific genomic locus, either on its own or as part of a complex. Coactivators often act by altering chromatin structure and modifications. For example, one class of transcription coactivators modifies chromatin structure through covalent modification of histones. A second class remodels the conformation of chromatin in an ATP-dependent fashion. A third class modulates interactions of DNA-bound DNA-binding transcription factors with other transcription coregulators. A fourth class of coactivator activity is the bridging of a DNA-binding transcription factor to the general (basal) transcription machinery. The Mediator complex, which bridges sequence-specific DNA binding transcription factors and RNA polymerase, is also a transcription coactivator. References: PMID:10213677, PMID:16858867 Sources: GOC:txnOH-2018 Also known as: transcription co-activator activity, RNA polymerase II transcription co-activator activity, RNA polymerase II transcription coactivator activity, RNA polymerase II transcription mediator activity